{
  "term_label": "nucleus",
  "gene_symbol": "MAPK10",
  "gene": "UniProtKB:P53779",
  "gene_name": "Mitogen-activated protein kinase 10",
  "term_id": "GO:0005634"
}